{
  "gene_name": "Peroxisomal membrane protein 4",
  "term_id": "GO:0005778",
  "gene": "UniProtKB:Q9Y6I8",
  "gene_symbol": "PXMP4",
  "term_label": "peroxisomal membrane"
}